{
  "gene_symbol": "LCN2",
  "term_label": "Unknown molecular function",
  "gene_name": "Neutrophil gelatinase-associated lipocalin",
  "gene": "UniProtKB:P80188",
  "term_id": "UNKNOWN:0001"
}